guanine deglycation, glyoxal removal [GO:0106046] (biological process) References: PMID:28596309 Relationships: is a type of guanine deglycation [GO:0106044] Definition: The removal of glyoxal from a glycated guanine, to form glycolate and a deglycated guanine.